striated muscle myosin thick filament [GO:0005863] (cellular component) Relationships: is a type of myosin filament [GO:0032982]; is a type of myofilament [GO:0036379]; is part of sarcomere [GO:0030017]; has part muscle myosin complex [GO:0005859] Definition: Bipolar filaments formed of polymers of a muscle-specific myosin II isoform, found in the middle of sarcomeres in myofibrils. Sources: GOC:mtg_muscle, ISBN:0815316194